{
  "gene_name": "Zinc finger protein 488",
  "term_id": "GO:0014003",
  "term_label": "oligodendrocyte development",
  "gene_symbol": "ZNF488",
  "gene": "UniProtKB:Q96MN9"
}